{
  "gene_symbol": "GRIK4",
  "gene": "UniProtKB:Q16099",
  "term_id": "GO:0042734",
  "gene_name": "Glutamate receptor ionotropic, kainate 4",
  "term_label": "presynaptic membrane"
}